octopamine dehydratase activity [GO:0050202] (molecular function) Also known as: octopamine hydro-lyase (deaminating), octopamine hydro-lyase [deaminating; (4-hydroxyphenyl)acetaldehyde-forming], octopamine hydrolyase activity Sources: EC:4.2.1.87, RHEA:18173 Definition: Catalysis of the reaction: 1-(4-hydroxyphenyl)-2-aminoethanol = (4-hydroxyphenyl)acetaldehyde + NH4. Relationships: is_a hydro-lyase activity [GO:0016836]